{
  "gene": "UniProtKB:Q9P2K9",
  "term_label": "Unknown molecular function",
  "gene_symbol": "DISP3",
  "term_id": "UNKNOWN:0001",
  "gene_name": "Protein dispatched homolog 3"
}